regulation of erythrocyte clearance [GO:0034106] (biological process) Subtypes: negative regulation of erythrocyte clearance [GO:0034107], positive regulation of erythrocyte clearance [GO:0034108] References: PMID:12905029, PMID:14754397 Sources: GOC:add Definition: Any process that modulates the frequency, rate, or extent of erythrocyte clearance. Relationships: is_a GO:0034103; regulates GO:0034102 Also known as: regulation of RBC clearance, regulation of red blood cell clearance, regulation of neocytolysis